{
  "term_id": "UNKNOWN:0001",
  "gene": "UniProtKB:Q8N4L4",
  "gene_symbol": "SPEM1",
  "gene_name": "Spermatid maturation protein 1",
  "term_label": "Unknown molecular function"
}